integrin alphav-beta6 complex [GO:0034685] (cellular component) Definition: An integrin complex that comprises one alphav subunit and one beta6 subunit. Relationships: is a type of integrin complex [GO:0008305] References: PMID:12297042 Also known as: alphav-beta6 integrin complex, ITGAV-ITGB6 complex